{
  "gene_symbol": "ZDHHC19",
  "term_label": "endoplasmic reticulum",
  "term_id": "GO:0005783",
  "gene": "UniProtKB:Q8WVZ1",
  "gene_name": "Palmitoyltransferase ZDHHC19"
}